cellular response to thyroid hormone stimulus [GO:0097067] (BP) References: PMID:9916872 Sources: GOC:sjw Definition: A change in state or activity of a cell (in terms of movement, secretion, enzyme production, gene expression, etc.) as a result of a thyroid hormone stimulus. Subtypes: cellular response to thyroxine stimulus [GO:0097069] Relationships: is a type of cellular response to hormone stimulus [GO:0032870]; is_a response to thyroid hormone [GO:0097066]